{
  "gene_name": "Pigment epithelium-derived factor",
  "term_label": "negative regulation of angiogenesis",
  "gene": "UniProtKB:P36955",
  "gene_symbol": "SERPINF1",
  "term_id": "GO:0016525"
}